hexaprenyl diphosphate synthase (geranylgeranyl-diphosphate specific) activity [GO:0052922] (molecular function) Sources: RHEA:27555 Also known as: (all-E) hexaprenyl diphosphate synthase activity, (all-trans)-hexaprenyl-diphosphate synthase activity, hexaprenyl diphosphate synthase activity, hexaprenyl pyrophosphate synthetase activity Definition: Catalysis of the reaction: 2 isopentenyl diphosphate + (2E,6E,10E)-geranylgeranyl diphosphate = all-trans-hexaprenyl diphosphate + 2 diphosphate. Relationships: is a type of GO:0120531